{
  "gene": "UniProtKB:P06126",
  "gene_name": "T-cell surface glycoprotein CD1a",
  "term_id": "GO:0030883",
  "term_label": "endogenous lipid antigen binding",
  "gene_symbol": "CD1A"
}